{
  "term_id": "GO:0007617",
  "gene": "UniProtKB:P07101",
  "term_label": "mating behavior",
  "gene_name": "Tyrosine 3-monooxygenase",
  "gene_symbol": "TH"
}